RGS6-DNMT1-DMAP1 complex [GO:0070313] (CC) References: PMID:14734556 Sources: GOC:mah Definition: A protein complex formed by the association of RGS6, a negative regulator of heterotrimeric G protein signaling, with the DMAP1-Dnmt1 transcriptional repressor complex; in the complex, RGS6 inhibits the transcriptional repressor activity of DMAP1. Relationships: is a type of nuclear protein-containing complex [GO:0140513]